{
  "term_id": "UNKNOWN:0001",
  "term_label": "Unknown molecular function",
  "gene_name": "SEC14-like protein 5",
  "gene_symbol": "SEC14L5",
  "gene": "UniProtKB:O43304"
}